{
  "gene": "UniProtKB:Q15554",
  "term_label": "double-stranded telomeric DNA binding",
  "gene_symbol": "TERF2",
  "term_id": "GO:0003691",
  "gene_name": "Telomeric repeat-binding factor 2"
}